auxin receptor activity [GO:0038198] (molecular function) Definition: Combining with auxin and transmitting the signal in the cell to initiate a change in cell activity. Auxin is a plant hormone (phytohormone). References: PMID:15917797 Sources: GOC:signaling Relationships: is a type of signaling receptor activity [GO:0038023]; is part of auxin-activated signaling pathway [GO:0009734]; has part auxin binding [GO:0010011]